protein deglycosylation [GO:0006517] (biological process) Definition: The removal of sugar residues from a glycosylated protein. Subtypes: protein deglycosylation involved in glycoprotein catabolic process [GO:0035977], protein demannosylation [GO:0036507] Also known as: glycoprotein deglycosylation Sources: GOC:mah Relationships: is a type of glycoprotein metabolic process [GO:0009100]; is a type of protein modification process [GO:0036211]